{
  "term_label": "serine import into mitochondrion",
  "gene_symbol": "SFXN1",
  "gene_name": "Sideroflexin-1",
  "gene": "UniProtKB:Q9H9B4",
  "term_id": "GO:0140300"
}